calcitonin gene-related peptide receptor signaling pathway [GO:1990408] (biological process) Definition: The series of molecular signals initiated by an extracellular calcitonin gene-related peptide (CGRP) combining with a calcitonin gene-related peptide receptor on the surface of the target cell. Calcitonin gene-related peptide receptors may form dimers, trimers or tetramers. References: PMID:10882736 Sources: GOC:bhm Note: An example of a protein that could be annotated to this term is CALCRL in human (Q16602) in PMID:10882736. Also known as: CGRP receptor signaling pathway, calcitonin-gene-related peptide receptor signaling pathway, calcitonin-gene-related polypeptide receptor signaling pathway Relationships: is a type of calcitonin family receptor signaling pathway [GO:0097646]